{
  "gene_name": "Pre-mRNA-processing factor 39",
  "term_id": "GO:0000243",
  "gene": "UniProtKB:Q86UA1",
  "term_label": "commitment complex",
  "gene_symbol": "PRPF39"
}